{
  "term_label": "nucleus",
  "term_id": "GO:0005634",
  "gene_symbol": "PUS3",
  "gene_name": "tRNA pseudouridine(38_39) synthase",
  "gene": "UniProtKB:Q9BZE2"
}